{
  "term_id": "GO:0000340",
  "term_label": "RNA 7-methylguanosine cap binding",
  "gene": "UniProtKB:Q7L576",
  "gene_name": "Cytoplasmic FMR1-interacting protein 1",
  "gene_symbol": "CYFIP1"
}